membrane assembly [GO:0071709] (BP) Definition: The aggregation, arrangement and bonding together of a set of components to form a membrane. Sources: GOC:mah Relationships: is a type of GO:0022607; is_a membrane organization [GO:0061024]; is part of membrane biogenesis [GO:0044091] Subtypes: GO:0001765, nuclear membrane reassembly [GO:0031468], ascospore-type prospore membrane formation [GO:0032120], Gram-negative-bacterium-type cell outer membrane assembly [GO:0043165], postsynaptic membrane assembly [GO:0097104], GO:0097105, GO:1903575